regulation of CD4-positive, alpha-beta T cell activation [GO:2000514] (biological process) Definition: Any process that modulates the frequency, rate or extent of CD4-positive, alpha-beta T cell activation. Sources: GOC:obol Relationships: is a type of regulation of alpha-beta T cell activation [GO:0046634]; regulates CD4-positive, alpha-beta T cell activation [GO:0035710] Subtypes: regulation of CD4-positive, alpha-beta T cell differentiation [GO:0043370], regulation of CD4-positive, alpha-beta T cell costimulation [GO:1900279], negative regulation of CD4-positive, alpha-beta T cell activation [GO:2000515], positive regulation of CD4-positive, alpha-beta T cell activation [GO:2000516], regulation of T-helper 1 cell activation [GO:2000517], regulation of CD4-positive, alpha-beta T cell proliferation [GO:2000561], regulation of T-helper 2 cell activation [GO:2000569]